{
  "gene": "UniProtKB:P01275",
  "gene_name": "Pro-glucagon",
  "gene_symbol": "GCG",
  "term_label": "hormone activity",
  "term_id": "GO:0005179"
}